{
  "gene": "UniProtKB:O75355",
  "gene_name": "Ectonucleoside triphosphate diphosphohydrolase 3",
  "term_id": "GO:0005886",
  "gene_symbol": "ENTPD3",
  "term_label": "plasma membrane"
}